{
  "gene_name": "Importin subunit alpha-8",
  "gene": "UniProtKB:A9QM74",
  "term_label": "NLS-bearing protein import into nucleus",
  "term_id": "GO:0006607",
  "gene_symbol": "KPNA7"
}